{
  "term_id": "GO:0005125",
  "gene_symbol": "MIF",
  "term_label": "cytokine activity",
  "gene_name": "Macrophage migration inhibitory factor",
  "gene": "UniProtKB:P14174"
}